{
  "gene_name": "Hexokinase-4",
  "term_id": "GO:0005739",
  "term_label": "mitochondrion",
  "gene": "UniProtKB:P35557",
  "gene_symbol": "GCK"
}